cell surface receptor signaling pathway [GO:0007166] (biological process) Subtypes: immune response-regulating cell surface receptor signaling pathway [GO:0002768], enzyme-linked receptor protein signaling pathway [GO:0007167], GO:0007215, Notch signaling pathway [GO:0007219], smoothened signaling pathway [GO:0007224], integrin-mediated signaling pathway [GO:0007229], Toll signaling pathway [GO:0008063], brassinosteroid mediated signaling pathway [GO:0009742], GO:0016055, cytokine-mediated signaling pathway [GO:0019221], CD40 signaling pathway [GO:0023035], lipopolysaccharide-mediated signaling pathway [GO:0031663], positive regulation of integrin activation by cell surface receptor linked signal transduction [GO:0033626], GO:0035385, purinergic nucleotide receptor signaling pathway [GO:0035590], Fas signaling pathway [GO:0036337], netrin-activated signaling pathway [GO:0038007], reelin-mediated signaling pathway [GO:0038026], apolipoprotein A-I-mediated signaling pathway [GO:0038027], GO:0038065, neurotrophin signaling pathway [GO:0038179], GO:0038184, neuropilin signaling pathway [GO:0038189], GO:0038195, cell surface receptor signaling pathway involved in heart development [GO:0061311], semaphorin-plexin signaling pathway [GO:0071526], GO:0097191, cell surface receptor signaling pathway via STAT [GO:0097696], GO:0099565, Norrin signaling pathway [GO:0110135], GO:0160162, beta-arrestin-dependent dopamine receptor signaling pathway [GO:0160213] Also known as: cell surface receptor linked signal transduction, cell surface receptor linked signaling pathway, cell surface receptor linked signalling pathway Sources: GOC:signaling Definition: The series of molecular signals initiated by an extracellular ligand binding to a receptor located on the cell surface. The pathway ends with regulation of a downstream cellular process, e.g. transcription. Relationships: is a type of GO:0007165